{
  "gene_symbol": "KCNJ4",
  "gene_name": "Inward rectifier potassium channel 4",
  "term_id": "UNKNOWN:0001",
  "gene": "UniProtKB:P48050",
  "term_label": "Unknown molecular function"
}